{
  "term_id": "GO:0030018",
  "term_label": "Z disc",
  "gene": "UniProtKB:P20929",
  "gene_name": "Nebulin",
  "gene_symbol": "NEB"
}